{
  "term_id": "UNKNOWN:0001",
  "gene_symbol": "TBC1D28",
  "gene_name": "TBC1 domain family member 28",
  "gene": "UniProtKB:Q2M2D7",
  "term_label": "Unknown molecular function"
}